{
  "gene": "UniProtKB:Q9NQ60",
  "gene_symbol": "EQTN",
  "term_label": "endocytosis",
  "gene_name": "Equatorin",
  "term_id": "GO:0006897"
}